plasma membrane electron transport, NADH to quinone [GO:0030965] (biological process) Relationships: is_a respiratory electron transport chain [GO:0022904]; is part of plasma membrane ATP synthesis coupled electron transport [GO:0042774] Definition: The transfer of electrons from NADH to the quinone pool that occurs during oxidative phosphorylation and results in the generation of a proton gradient, mediated by the enzyme known as NADH-quinone oxidoreductase. Sources: GOC:mah, GOC:sd